{
  "term_label": "Unknown cellular component",
  "gene_symbol": "CCDC51",
  "gene_name": "Mitochondrial potassium channel",
  "gene": "UniProtKB:Q96ER9",
  "term_id": "UNKNOWN:0003"
}